{
  "gene": "UniProtKB:P50135",
  "term_id": "GO:0005829",
  "term_label": "cytosol",
  "gene_name": "Histamine N-methyltransferase",
  "gene_symbol": "HNMT"
}